microtubule end [GO:1990752] (cellular component) Sources: GOC:pr Subtypes: microtubule plus-end [GO:0035371], GO:0036449, mitotic spindle astral microtubule end [GO:1905721], post-anaphase array microtubule end [GO:1905760] Definition: Any end of a microtubule. Microtubule ends differ in that the so-called microtubule plus-end is the one that preferentially grows by polymerization, with respect to the minus-end. Note: This term should be used when it is not possible to distinguish between the two microtubule ends, e.g. during image annotation. Whenever possible, please annotate to one of the more specific children GO:0035371 'microtubule plus-end' or GO:0036449 'microtubule minus-end'. Relationships: is a type of cellular anatomical structure [GO:0110165]; is part of GO:0005874